{
  "gene_symbol": "SHC2",
  "term_label": "plasma membrane",
  "gene_name": "SHC-transforming protein 2",
  "gene": "UniProtKB:P98077",
  "term_id": "GO:0005886"
}